{
  "term_id": "UNKNOWN:0001",
  "gene_symbol": "UQCC3",
  "term_label": "Unknown molecular function",
  "gene": "UniProtKB:Q6UW78",
  "gene_name": "Ubiquinol-cytochrome-c reductase complex assembly factor 3"
}